{
  "term_label": "Notch receptor processing",
  "gene": "UniProtKB:Q96BI3",
  "term_id": "GO:0007220",
  "gene_symbol": "APH1A",
  "gene_name": "Gamma-secretase subunit APH-1A"
}